{
  "term_label": "nucleus",
  "gene_name": "Zinc finger CCHC domain-containing protein 18",
  "gene": "UniProtKB:P0CG32",
  "term_id": "GO:0005634",
  "gene_symbol": "ZCCHC18"
}